{
  "gene_symbol": "PRR19",
  "term_label": "Unknown cellular component",
  "gene_name": "Proline-rich protein 19",
  "term_id": "UNKNOWN:0003",
  "gene": "UniProtKB:A6NJB7"
}